nitrite efflux transmembrane transporter activity [GO:0015514] (molecular function) Sources: GOC:mtg_transport, ISBN:0815340729 Definition: Enables the transfer of nitrite from the inside of the cell to the outside of the cell across a membrane. Relationships: is a type of nitrite transmembrane transporter activity [GO:0015113]; is a type of GO:0015291; is a type of efflux transmembrane transporter activity [GO:0015562] Also known as: nitrite extrusion permease activity